{
  "term_label": "nucleus",
  "gene_symbol": "MYG1",
  "gene_name": "MYG1 exonuclease",
  "gene": "UniProtKB:Q9HB07",
  "term_id": "GO:0005634"
}